{
  "term_label": "Unknown molecular function",
  "gene_symbol": "GPATCH11",
  "gene_name": "G patch domain-containing protein 11",
  "term_id": "UNKNOWN:0001",
  "gene": "UniProtKB:Q8N954"
}